{
  "term_label": "synaptic vesicle membrane",
  "term_id": "GO:0030672",
  "gene_symbol": "SYT1",
  "gene_name": "Synaptotagmin-1",
  "gene": "UniProtKB:P21579"
}